{
  "gene": "UniProtKB:P40259",
  "gene_symbol": "CD79B",
  "gene_name": "B-cell antigen receptor complex-associated protein beta chain",
  "term_id": "GO:0004888",
  "term_label": "transmembrane signaling receptor activity"
}